{
  "gene_symbol": "SKP1",
  "term_label": "cullin family protein binding",
  "term_id": "GO:0097602",
  "gene_name": "S-phase kinase-associated protein 1",
  "gene": "UniProtKB:P63208"
}